{
  "term_label": "coenzyme A diphosphatase activity",
  "gene": "UniProtKB:Q8WV74",
  "term_id": "GO:0010945",
  "gene_name": "Mitochondrial coenzyme A diphosphatase NUDT8",
  "gene_symbol": "NUDT8"
}